medulla oblongata structural organization [GO:0021581] (biological process) Sources: GOC:cls, GOC:dgh, GOC:dph, GOC:jid, GO_REF:0000021 Also known as: medulla oblongata structural organisation, medulla structural maturation, myelencephalon structural maturation Relationships: is a type of anatomical structure arrangement [GO:0048532]; is part of GO:0021577; is part of medulla oblongata morphogenesis [GO:0021579] Definition: The process that contributes to the act of creating the structural organization of the medulla oblongata. This process pertains to the physical shaping of a rudimentary structure. The medulla oblongata lies directly above the spinal cord and controls vital autonomic functions such as digestion, breathing and the control of heart rate.